{
  "gene": "UniProtKB:Q76KX8",
  "gene_symbol": "ZNF534",
  "gene_name": "Zinc finger protein 534",
  "term_label": "DNA-binding transcription factor activity, RNA polymerase II-specific",
  "term_id": "GO:0000981"
}